endothelial cell proliferation [GO:0001935] (biological process) Definition: The multiplication or reproduction of endothelial cells, resulting in the expansion of a cell population. Endothelial cells are thin flattened cells which line the inside surfaces of body cavities, blood vessels, and lymph vessels, making up the endothelium. Relationships: is a type of epithelial cell proliferation [GO:0050673] Sources: GOC:add, ISBN:0781735149 Regulation: regulated by regulation of endothelial cell proliferation [GO:0001936]; negatively regulated by negative regulation of endothelial cell proliferation [GO:0001937]; positively regulated by positive regulation of endothelial cell proliferation [GO:0001938] Subtypes: blood vessel endothelial cell proliferation involved in sprouting angiogenesis [GO:0002043], vascular endothelial cell proliferation [GO:0101023]